{
  "gene": "UniProtKB:Q8TDQ7",
  "gene_symbol": "GNPDA2",
  "term_label": "N-acetylneuraminate catabolic process",
  "term_id": "GO:0019262",
  "gene_name": "Glucosamine-6-phosphate isomerase 2"
}